{
  "term_label": "Unknown biological process",
  "gene": "UniProtKB:C9J6K1",
  "term_id": "UNKNOWN:0002",
  "gene_symbol": "C19orf81",
  "gene_name": "Putative uncharacterized protein C19orf81"
}